{
  "gene_symbol": "GPRC5C",
  "gene": "UniProtKB:Q9NQ84",
  "term_id": "GO:0043235",
  "term_label": "receptor complex",
  "gene_name": "G-protein coupled receptor family C group 5 member C"
}